ADP-sugar diphosphatase activity [GO:0019144] (molecular function) Definition: Catalysis of the reaction: ADP-sugar + H2O = AMP + sugar 1-phosphate. Sources: EC:3.6.1.21 Also known as: nucleoside diphosphate-sugar hydrolase activity, ADP-sugar pyrophosphatase activity, ADP-sugar sugarphosphohydrolase activity, ADPsugar pyrophosphatase activity, adenosine diphosphosugar pyrophosphatase activity Relationships: is a type of GO:0016462 Subtypes: ADP-ribose pyrophosphohydrolase activity [GO:0080041], ADP-glucose pyrophosphohydrolase activity [GO:0080042]